negative regulation of organofluorine metabolic process [GO:0090350] (biological process) Definition: Any process that decreases the rate, frequency or extent of the chemical reactions and pathways involving organofluorine compounds, as carried out by individual cells. Sources: GOC:BHF Relationships: is a type of negative regulation of metabolic process [GO:0009892]; is a type of regulation of organohalogen metabolic process [GO:0090347]; negatively regulates organofluorine metabolic process [GO:0090346]